cardiac muscle cell fate commitment [GO:0060923] (biological process) Sources: GOC:mtg_heart Also known as: cardiomyocyte cell fate commitment, heart muscle cell fate commitment Definition: The commitment of cells to specific cardiac muscle cell fates and their capacity to differentiate into cardiac muscle cells. Cardiac muscle cells are striated muscle cells that are responsible for heart contraction. Relationships: is a type of muscle cell fate commitment [GO:0042693]; is a type of cardiac cell fate commitment [GO:0060911]; is part of cardiac muscle cell differentiation [GO:0055007] Subtypes: GO:0060924, ventricular cardiac muscle cell fate commitment [GO:0060925], cardiac pacemaker cell fate commitment [GO:0060927]